{
  "gene_name": "Cell cycle exit and neuronal differentiation protein 1",
  "term_label": "Unknown molecular function",
  "term_id": "UNKNOWN:0001",
  "gene": "UniProtKB:Q8N111",
  "gene_symbol": "CEND1"
}